vesicle fusion with vesicle [GO:0061782] (biological process) Also known as: vesicle to vesicle fusion, vesicle-vesicle fusion Relationships: is a type of GO:0006906 References: PMID:16618809 Sources: GOC:PARL, GOC:bf Definition: Fusion of the membrane of a transport vesicle with a target membrane on another vesicle.